{
  "gene_name": "Copper-transporting ATPase 1",
  "gene": "UniProtKB:Q04656",
  "term_label": "trans-Golgi network",
  "gene_symbol": "ATP7A",
  "term_id": "GO:0005802"
}